{
  "gene": "UniProtKB:P37173",
  "term_label": "plasma membrane",
  "gene_name": "TGF-beta receptor type-2",
  "gene_symbol": "TGFBR2",
  "term_id": "GO:0005886"
}